{
  "gene_name": "Centrosomal protein of 192 kDa",
  "gene_symbol": "CEP192",
  "gene": "UniProtKB:Q8TEP8",
  "term_label": "Unknown molecular function",
  "term_id": "UNKNOWN:0001"
}